{
  "term_label": "Unknown cellular component",
  "gene_symbol": "Q5PR19",
  "gene_name": "Putative UPF0607 protein LOC392364",
  "term_id": "UNKNOWN:0003",
  "gene": "UniProtKB:Q5PR19"
}